dTMP biosynthetic process [GO:0006231] (BP) Sources: ISBN:0198506732 Subtypes: dTMP salvage [GO:0036198] Relationships: is a type of GO:0009177; is a type of pyrimidine deoxyribonucleotide biosynthetic process [GO:0009221]; is a type of dTMP metabolic process [GO:0046073] Also known as: dTMP anabolism, dTMP biosynthesis, dTMP formation, dTMP synthesis Definition: The chemical reactions and pathways resulting in the formation of dTMP, deoxyribosylthymine monophosphate (2'-deoxyribosylthymine 5'-phosphate).